{
  "term_id": "UNKNOWN:0003",
  "term_label": "Unknown cellular component",
  "gene_symbol": "ERICH1",
  "gene": "UniProtKB:Q86X53",
  "gene_name": "Glutamate-rich protein 1"
}